{
  "gene": "UniProtKB:O00189",
  "gene_symbol": "AP4M1",
  "term_label": "AP-1 adaptor complex",
  "term_id": "GO:0030121",
  "gene_name": "AP-4 complex subunit mu-1"
}